23S rRNA pseudouridine(746) synthase activity [GO:0160142] (molecular function) Sources: EC:5.4.99.29, RHEA:42548 Relationships: is a type of rRNA pseudouridine synthase activity [GO:0120159] Definition: Catalysis of the reaction: uridine(746) in 23S rRNA = pseudouridine(746) in 23S rRNA.